negative regulation of spindle assembly [GO:1905831] (BP) Relationships: is a type of negative regulation of cell cycle process [GO:0010948]; is a type of negative regulation of cytoskeleton organization [GO:0051494]; is a type of GO:0090169; is a type of negative regulation of organelle assembly [GO:1902116]; negatively regulates GO:0051225 Subtypes: negative regulation of mitotic spindle formation (spindle phase one) [GO:0110160] Also known as: down regulation of bipolar spindle biosynthesis, down regulation of bipolar spindle formation, down regulation of spindle assembly, down regulation of spindle biosynthesis, down regulation of spindle formation, down-regulation of bipolar spindle biosynthesis, down-regulation of bipolar spindle formation, down-regulation of spindle assembly, down-regulation of spindle biosynthesis, down-regulation of spindle formation, downregulation of bipolar spindle biosynthesis, downregulation of bipolar spindle formation, downregulation of spindle assembly, downregulation of spindle biosynthesis, downregulation of spindle formation, negative regulation of bipolar spindle biosynthesis, negative regulation of bipolar spindle formation, negative regulation of spindle biosynthesis, negative regulation of spindle formation, inhibition of bipolar spindle biosynthesis, inhibition of bipolar spindle formation, inhibition of spindle assembly, inhibition of spindle biosynthesis, inhibition of spindle formation References: PMID:27689799 Sources: GOC:TermGenie, GO_REF:0000058 Definition: Any process that stops, prevents or reduces the frequency, rate or extent of spindle assembly.